{
  "gene_name": "Transcription factor RelB",
  "gene_symbol": "RELB",
  "term_id": "GO:0038061",
  "term_label": "non-canonical NF-kappaB signal transduction",
  "gene": "UniProtKB:Q01201"
}